{
  "term_id": "GO:0004382",
  "gene": "UniProtKB:Q9Y227",
  "gene_name": "Ectonucleoside triphosphate diphosphohydrolase 4",
  "gene_symbol": "ENTPD4",
  "term_label": "GDP phosphatase activity"
}